protein-containing complex assembly involved in synapse maturation [GO:0090126] (biological process) Sources: GOC:ascb_2009, GOC:dph, GOC:tb Also known as: protein complex assembly involved in synapse maturation Relationships: is a type of protein-containing complex assembly [GO:0065003]; is part of synapse maturation [GO:0060074] Definition: The aggregation, arrangement and bonding together of a set of components to form a protein complex that contributes to synapse maturation.